carbohydrate derivative metabolic process [GO:1901135] (BP) Subtypes: fructose 6-phosphate metabolic process [GO:0006002], fructose 2,6-bisphosphate metabolic process [GO:0006003], aminoglycan metabolic process [GO:0006022], amino sugar metabolic process [GO:0006040], GO:0009051, glycoprotein metabolic process [GO:0009100], nucleoside metabolic process [GO:0009116], GO:0009225, deoxyribonucleotide metabolic process [GO:0009262], glycoside metabolic process [GO:0016137], GO:0019255, sucrose catabolic process via 3'-ketosucrose [GO:0019574], GO:0019682, ribose phosphate metabolic process [GO:0019693], GO:0019760, fructose 1,6-bisphosphate metabolic process [GO:0030388], teichoic acid metabolic process [GO:0046374], K antigen metabolic process [GO:0046375], GO:0046377, GO:0046378, GO:0051156, GO:0051167, alditol phosphate metabolic process [GO:0052646], GO:0052778, chitobiose catabolic process [GO:0052781], glycerol to glycerone phosphate metabolic process [GO:0061610], GO:1901136, GO:1901137, lipooligosaccharide metabolic process [GO:1901269], GO:1903509, amylopectin metabolic process [GO:2000896], GO:2001060 Also known as: carbohydrate derivative metabolism Definition: The chemical reactions and pathways involving carbohydrate derivative. Sources: GOC:TermGenie Relationships: is a type of metabolic process [GO:0008152]